{
  "gene_symbol": "FFAR1",
  "gene_name": "Free fatty acid receptor 1",
  "gene": "UniProtKB:O14842",
  "term_label": "bioactive lipid receptor activity",
  "term_id": "GO:0045125"
}